{
  "term_id": "GO:0007268",
  "gene_name": "Solute carrier family 12 member 7",
  "gene_symbol": "SLC12A7",
  "gene": "UniProtKB:Q9Y666",
  "term_label": "chemical synaptic transmission"
}